{
  "gene_name": "Kinetochore protein Nuf2",
  "gene_symbol": "NUF2",
  "gene": "UniProtKB:Q9BZD4",
  "term_id": "GO:0045132",
  "term_label": "meiotic chromosome segregation"
}